{
  "term_id": "GO:0031430",
  "gene_name": "Myosin-binding protein C, slow-type",
  "gene_symbol": "MYBPC1",
  "gene": "UniProtKB:Q00872",
  "term_label": "M band"
}